{
  "term_id": "GO:0071006",
  "gene": "UniProtKB:Q9UMS4",
  "term_label": "U2-type catalytic step 1 spliceosome",
  "gene_name": "Pre-mRNA-processing factor 19",
  "gene_symbol": "PRPF19"
}